{
  "gene_name": "Zinc finger CCCH domain-containing protein 11B",
  "gene_symbol": "ZC3H11B",
  "term_id": "GO:0016973",
  "term_label": "poly(A)+ mRNA export from nucleus",
  "gene": "UniProtKB:A0A1B0GTU1"
}